occurs in [BFO:0000066] (external)